{
  "gene": "UniProtKB:P62993",
  "term_label": "plasma membrane",
  "gene_symbol": "GRB2",
  "gene_name": "Growth factor receptor-bound protein 2",
  "term_id": "GO:0005886"
}